{
  "gene_name": "Vesicle transport through interaction with t-SNAREs homolog 1A",
  "gene_symbol": "VTI1A",
  "term_label": "vesicle fusion with Golgi apparatus",
  "gene": "UniProtKB:Q96AJ9",
  "term_id": "GO:0048280"
}